endothelial tube lumen extension involved in blood vessel lumen ensheathment [GO:1902355] (biological process) Definition: Any endothelial tube lumen extension that is involved in blood vessel lumen ensheathment. References: PMID:23698350 Sources: GOC:TermGenie, GOC:dgh Relationships: is a type of GO:0097498; BFO_0000050 blood vessel lumen ensheathment [GO:0097496]